{
  "term_id": "GO:0099634",
  "term_label": "postsynaptic specialization membrane",
  "gene_name": "Neuroligin-2",
  "gene": "UniProtKB:Q8NFZ4",
  "gene_symbol": "NLGN2"
}